{
  "gene_symbol": "NR0B1",
  "gene": "UniProtKB:P51843",
  "term_id": "GO:0005737",
  "term_label": "cytoplasm",
  "gene_name": "Nuclear receptor subfamily 0 group B member 1"
}